{
  "gene_name": "Protein phosphatase 1F",
  "term_label": "positive regulation of stress fiber assembly",
  "term_id": "GO:0051496",
  "gene": "UniProtKB:P49593",
  "gene_symbol": "PPM1F"
}